{
  "gene": "UniProtKB:Q96KT7",
  "gene_name": "Solute carrier family 35 member G5",
  "gene_symbol": "SLC35G5",
  "term_id": "UNKNOWN:0002",
  "term_label": "Unknown biological process"
}